lipopolysaccharide metabolic process [GO:0008653] (biological process) Definition: The chemical reactions and pathways involving lipopolysaccharides, a group of related, structurally complex components of the outer membrane of Gram-negative bacteria. Lipopolysaccharides consist three covalently linked regions, lipid A, core oligosaccharide, and an O side chain. Lipid A is responsible for the toxicity of the lipopolysaccharide. Sources: ISBN:0198506732 Also known as: LPS metabolic process, lipopolysaccharide metabolism Relationships: is a type of macromolecule metabolic process [GO:0043170]; is a type of GO:1903509 Subtypes: lipopolysaccharide biosynthetic process [GO:0009103], GO:0009104